{
  "gene_symbol": "TC2N",
  "term_id": "UNKNOWN:0001",
  "term_label": "Unknown molecular function",
  "gene_name": "Tandem C2 domains nuclear protein",
  "gene": "UniProtKB:Q8N9U0"
}